{
  "term_id": "UNKNOWN:0002",
  "gene_symbol": "SLX9",
  "gene_name": "Ribosome biogenesis protein SLX9 homolog",
  "term_label": "Unknown biological process",
  "gene": "UniProtKB:Q9NSI2"
}